{
  "gene": "UniProtKB:O75582",
  "term_id": "GO:0038202",
  "gene_name": "Ribosomal protein S6 kinase alpha-5",
  "term_label": "TORC1 signaling",
  "gene_symbol": "RPS6KA5"
}